{
  "term_id": "GO:0005737",
  "gene": "UniProtKB:Q9Y6E0",
  "gene_name": "Serine_threonine-protein kinase 24",
  "term_label": "cytoplasm",
  "gene_symbol": "STK24"
}